regulation of striated muscle cell differentiation [GO:0051153] (biological process) Subtypes: regulation of myotube differentiation [GO:0010830], GO:0051154, positive regulation of striated muscle cell differentiation [GO:0051155], regulation of cardiac muscle cell differentiation [GO:2000725] Sources: CL:0000737, GOC:ai Relationships: is a type of regulation of muscle cell differentiation [GO:0051147]; regulates GO:0051146 Definition: Any process that modulates the frequency, rate or extent of striated muscle cell differentiation.